{
  "term_id": "GO:0004490",
  "term_label": "methylglutaconyl-CoA hydratase activity",
  "gene": "UniProtKB:Q13825",
  "gene_symbol": "AUH",
  "gene_name": "Methylglutaconyl-CoA hydratase, mitochondrial"
}